sinoatrial valve formation [GO:0003194] (BP) Relationships: is a type of heart valve formation [GO:0003188]; is part of sinoatrial valve morphogenesis [GO:0003185] Also known as: SA valve formation Sources: GOC:mtg_heart Definition: The developmental process pertaining to the initial formation of the sinoatrial valve from unspecified parts. This process begins with the specific processes that contribute to the appearance of the discrete structure and ends when the structural rudiment is recognizable.